{
  "gene_symbol": "FAM106A",
  "term_label": "Unknown molecular function",
  "gene_name": "Protein FAM106A",
  "gene": "UniProtKB:Q4KMX7",
  "term_id": "UNKNOWN:0001"
}